{
  "term_label": "nucleus",
  "gene": "UniProtKB:Q8TBK2",
  "gene_name": "N-lysine methyltransferase SETD6",
  "term_id": "GO:0005634",
  "gene_symbol": "SETD6"
}